nitrite reductase (NO-forming) activity [GO:0050421] (molecular function) Sources: RHEA:15233 Definition: Catalysis of the reaction: nitric oxide + Fe(III)-[cytochrome c] + H2O = Fe(II)-[cytochrome c] + nitrite + 2 H+. Relationships: is a type of oxidoreductase activity, acting on other nitrogenous compounds as donors, cytochrome as acceptor [GO:0016662]; is a type of GO:0098809 Also known as: NO-forming nitrite reductase (cytochrome) activity, NO-forming nitrite reductase activity, cd-cytochrome nitrite reductase activity, cytochrome cd activity, cytochrome cd1 activity, methyl viologen-nitrite reductase activity, [nitrite reductase (cytochrome)], cytochrome c-551:O2, NO2(+) oxidoreductase activity, cytochrome c-551:O2, NO2+ oxidoreductase activity, nitric-oxide:ferricytochrome-c oxidoreductase activity, nitrite reductase (cytochrome; NO-forming) activity